positive regulation of ER to Golgi vesicle-mediated transport [GO:1902953] (biological process) Definition: Any process that activates or increases the frequency, rate or extent of ER to Golgi vesicle-mediated transport. Also known as: positive regulation of ER to Golgi transport, positive regulation of endoplasmic reticulum to Golgi transport, positive regulation of endoplasmic reticulum to Golgi vesicle-mediated transport, positive regulation of rough ER to cis-Golgi transport, positive regulation of rough ER to cis-Golgi vesicle-mediated transport, positive regulation of rough endoplasmic reticulum to cis-Golgi transport, positive regulation of rough endoplasmic reticulum to cis-Golgi vesicle-mediated transport, up regulation of ER to Golgi transport, up regulation of ER to Golgi vesicle-mediated transport, up regulation of endoplasmic reticulum to Golgi transport, up regulation of endoplasmic reticulum to Golgi vesicle-mediated transport, up regulation of rough ER to cis-Golgi transport, up regulation of rough ER to cis-Golgi vesicle-mediated transport, up regulation of rough endoplasmic reticulum to cis-Golgi transport, up regulation of rough endoplasmic reticulum to cis-Golgi vesicle-mediated transport, up-regulation of ER to Golgi transport, up-regulation of ER to Golgi vesicle-mediated transport, up-regulation of endoplasmic reticulum to Golgi transport, up-regulation of endoplasmic reticulum to Golgi vesicle-mediated transport, up-regulation of rough ER to cis-Golgi transport, up-regulation of rough ER to cis-Golgi vesicle-mediated transport, up-regulation of rough endoplasmic reticulum to cis-Golgi transport, up-regulation of rough endoplasmic reticulum to cis-Golgi vesicle-mediated transport, upregulation of ER to Golgi transport, upregulation of ER to Golgi vesicle-mediated transport, upregulation of endoplasmic reticulum to Golgi transport, upregulation of endoplasmic reticulum to Golgi vesicle-mediated transport, upregulation of rough ER to cis-Golgi transport, upregulation of rough ER to cis-Golgi vesicle-mediated transport, upregulation of rough endoplasmic reticulum to cis-Golgi transport, upregulation of rough endoplasmic reticulum to cis-Golgi vesicle-mediated transport, activation of ER to Golgi transport, activation of ER to Golgi vesicle-mediated transport, activation of endoplasmic reticulum to Golgi transport, activation of endoplasmic reticulum to Golgi vesicle-mediated transport, activation of rough ER to cis-Golgi transport, activation of rough ER to cis-Golgi vesicle-mediated transport, activation of rough endoplasmic reticulum to cis-Golgi transport, activation of rough endoplasmic reticulum to cis-Golgi vesicle-mediated transport Relationships: is a type of positive regulation of intracellular transport [GO:0032388]; is a type of GO:0060628; positively regulates endoplasmic reticulum to Golgi vesicle-mediated transport [GO:0006888] References: PMID:17855360 Sources: GOC:TermGenie, GOC:sjp, GO_REF:0000058